{
  "term_id": "GO:0005615",
  "gene_name": "Lactotransferrin",
  "term_label": "extracellular space",
  "gene_symbol": "LTF",
  "gene": "UniProtKB:P02788"
}